{
  "term_id": "GO:0060271",
  "gene_name": "Tektin-5",
  "gene": "UniProtKB:Q96M29",
  "term_label": "cilium assembly",
  "gene_symbol": "TEKT5"
}